{
  "gene_symbol": "OR6B2",
  "term_label": "olfactory receptor activity",
  "gene": "UniProtKB:Q6IFH4",
  "gene_name": "Olfactory receptor 6B2",
  "term_id": "GO:0004984"
}